positive regulation of mitotic chromosome condensation [GO:1903380] (biological process) Also known as: up regulation of mitotic chromosome condensation, up-regulation of mitotic chromosome condensation, upregulation of mitotic chromosome condensation, activation of mitotic chromosome condensation Relationships: is a type of positive regulation of cell cycle process [GO:0090068]; is a type of GO:1903379; is a type of GO:1905821; positively regulates mitotic chromosome condensation [GO:0007076] Definition: Any process that activates or increases the frequency, rate or extent of mitotic chromosome condensation. References: PMID:9490640 Sources: GOC:TermGenie, GO_REF:0000058